{
  "gene_name": "Terminal uridylyltransferase 7",
  "gene": "UniProtKB:Q5VYS8",
  "term_id": "GO:0031123",
  "gene_symbol": "TUT7",
  "term_label": "RNA 3'-end processing"
}